{
  "term_label": "histone binding",
  "term_id": "GO:0042393",
  "gene_symbol": "CHD7",
  "gene_name": "Chromodomain-helicase-DNA-binding protein 7",
  "gene": "UniProtKB:Q9P2D1"
}